membrane disassembly [GO:0030397] (biological process) Also known as: membrane breakdown, membrane catabolism, membrane degradation Definition: The controlled breakdown of any cell membrane in the context of a normal process such as autophagy. Subtypes: thylakoid membrane disassembly [GO:0010547], autophagosome membrane disassembly [GO:0030399], GO:0034496, sperm plasma membrane disassembly [GO:0035045], nuclear membrane disassembly [GO:0051081] Relationships: is a type of cellular component disassembly [GO:0022411]; is_a GO:0061024 Sources: GOC:mah Regulation: regulated by GO:0010549